negative regulation of B cell tolerance induction [GO:0002662] (biological process) Relationships: is a type of negative regulation of tolerance induction [GO:0002644]; is a type of GO:0002661; negatively regulates B cell tolerance induction [GO:0002514] Also known as: down regulation of B cell tolerance induction, down-regulation of B cell tolerance induction, downregulation of B cell tolerance induction, negative regulation of B lymphocyte tolerance induction, negative regulation of B-cell tolerance induction, negative regulation of B-lymphocyte tolerance induction, inhibition of B cell tolerance induction Subtypes: GO:0002671, GO:0002868, negative regulation of central B cell tolerance induction [GO:0002896] Sources: GOC:add Definition: Any process that stops, prevents, or reduces the frequency, rate, or extent of B cell tolerance induction.